{
  "gene": "UniProtKB:Q9NY87",
  "term_label": "Unknown biological process",
  "term_id": "UNKNOWN:0002",
  "gene_name": "Sperm protein associated with the nucleus on the X chromosome C",
  "gene_symbol": "SPANXC"
}